lipoprotein localization [GO:0044872] (BP) Definition: Any process in which a lipoprotein is transported to, or maintained in, a specific location. Sources: GOC:jl Relationships: is a type of GO:0033036 Subtypes: lipoprotein transport [GO:0042953], lipoprotein localization to membrane [GO:0044873]